{
  "gene": "UniProtKB:Q92564",
  "term_id": "GO:0045116",
  "term_label": "protein neddylation",
  "gene_symbol": "DCUN1D4",
  "gene_name": "DCN1-like protein 4"
}